{
  "gene": "UniProtKB:Q5T6S3",
  "term_label": "negative regulation of gene expression, epigenetic",
  "term_id": "GO:0045814",
  "gene_name": "PHD finger protein 19",
  "gene_symbol": "PHF19"
}